{
  "term_id": "GO:0003678",
  "term_label": "DNA helicase activity",
  "gene": "UniProtKB:Q96RR1",
  "gene_name": "Twinkle mtDNA helicase",
  "gene_symbol": "TWNK"
}